{
  "gene_symbol": "CALN1",
  "gene": "UniProtKB:Q9BXU9",
  "term_id": "GO:0032588",
  "term_label": "trans-Golgi network membrane",
  "gene_name": "Calcium-binding protein 8"
}